membrane depolarization during ventricular cardiac muscle cell action potential [GO:0098913] (biological process) Definition: The process in which ventricular cardiac muscle cell membrane potential changes in the depolarizing direction from the negative resting potential towards the positive membrane potential that will be the peak of the action potential. Relationships: is a type of GO:0086012; is part of GO:0086005 Sources: GOC:dph, GOC:mtg_cardiac_conduct_nov11, GOC:tb Also known as: electrocardiogram QRS complex, ventricular depolarization